{
  "gene_symbol": "DNM1L",
  "gene_name": "Dynamin-1-like protein",
  "term_label": "microtubule",
  "term_id": "GO:0005874",
  "gene": "UniProtKB:O00429"
}